{
  "term_label": "sensory perception of sound",
  "gene": "UniProtKB:O43405",
  "term_id": "GO:0007605",
  "gene_name": "Cochlin",
  "gene_symbol": "COCH"
}